{
  "gene_symbol": "WAC",
  "gene_name": "WW domain-containing adapter protein with coiled-coil",
  "term_id": "GO:0003682",
  "gene": "UniProtKB:Q9BTA9",
  "term_label": "chromatin binding"
}